{
  "term_id": "GO:0016567",
  "gene_symbol": "CUL3",
  "gene_name": "Cullin-3",
  "gene": "UniProtKB:Q13618",
  "term_label": "protein ubiquitination"
}